{
  "gene_name": "Neurofilament light polypeptide",
  "gene_symbol": "NEFL",
  "term_id": "GO:0033693",
  "term_label": "neurofilament bundle assembly",
  "gene": "UniProtKB:P07196"
}